{
  "term_label": "Unknown molecular function",
  "gene": "UniProtKB:Q86YD1",
  "gene_symbol": "PTOV1",
  "term_id": "UNKNOWN:0001",
  "gene_name": "Prostate tumor-overexpressed gene 1 protein"
}